{
  "term_id": "GO:0001786",
  "term_label": "phosphatidylserine binding",
  "gene": "UniProtKB:P08758",
  "gene_name": "Annexin A5",
  "gene_symbol": "ANXA5"
}